{
  "gene_symbol": "LALBA",
  "gene": "UniProtKB:P00709",
  "gene_name": "Alpha-lactalbumin",
  "term_id": "GO:0003796",
  "term_label": "lysozyme activity"
}